centriole replication [GO:0007099] (biological process) Regulation: regulated by regulation of centriole replication [GO:0046599]; negatively regulated by negative regulation of centriole replication [GO:0046600]; positively regulated by positive regulation of centriole replication [GO:0046601] Relationships: is a type of cell cycle process [GO:0022402]; is_a GO:0098534; is part of centrosome duplication [GO:0051298] Also known as: microtubule basal body duplication, centriole duplication, ciliary basal body duplication Definition: The cell cycle process in which a daughter centriole is formed perpendicular to an existing centriole. An immature centriole contains a ninefold radially symmetric array of single microtubules; mature centrioles consist of a radial array of nine microtubule triplets, doublets, or singlets depending upon the species and cell type. Duplicated centrioles also become the ciliary basal body in cells that form cilia during G0. References: PMID:9889124 Sources: GOC:cilia, GOC:kmv, ISBN:0815316194